cell migration involved in endocardial cushion formation [GO:0003273] (biological process) Sources: GOC:mtg_heart Definition: The orderly movement of a cell from one site to another that will contribute to the formation of an endocardial cushion. The endocardial cushion is a specialized region of mesenchymal cells that will give rise to the heart septa and valves. Relationships: is a type of cell migration involved in heart development [GO:0060973]; is part of endocardial cushion formation [GO:0003272]